interferon-kappa production [GO:0072649] (biological process) Relationships: is a type of type I interferon production [GO:0032606] Note: Note that this term is in the subset of terms that should not be used for direct gene product annotation. Instead, select one of the 'regulation' children terms. Also known as: IFN-kappa production, IFNK production, interferon-kappa secretion Definition: The appearance of interferon-kappa due to biosynthesis or secretion following a cellular stimulus, resulting in an increase in its intracellular or extracellular levels. References: PMID:15546383 Sources: GOC:BHF, GOC:mah